{
  "gene_symbol": "CASP9",
  "gene_name": "Caspase-9",
  "gene": "UniProtKB:P55211",
  "term_label": "cytosol",
  "term_id": "GO:0005829"
}